{
  "gene_symbol": "LGI2",
  "gene_name": "Leucine-rich repeat LGI family member 2",
  "term_label": "Unknown cellular component",
  "gene": "UniProtKB:Q8N0V4",
  "term_id": "UNKNOWN:0003"
}